{
  "term_id": "GO:0005739",
  "gene_symbol": "CISD3",
  "gene": "UniProtKB:P0C7P0",
  "term_label": "mitochondrion",
  "gene_name": "CDGSH iron-sulfur domain-containing protein 3, mitochondrial"
}